mitochondrial polycistronic RNA processing [GO:0140040] (biological process) Relationships: is a type of GO:0000963 Definition: The conversion of polycistronic RNA transcribed from a mitochondrial genome into mono- or bi-cistronic RNAs. References: PMID:20211597